GPCR sweet taste receptor activity [GO:0090683] (molecular function) Sources: GOC:hat, GOC:tb Also known as: G-protein coupled receptor sweet taste receptor activity Definition: A G protein-coupled receptor activity that is responsible for the sense of sweet taste. Relationships: is a type of sweet taste receptor activity [GO:0033041]; is a type of GPCR taste receptor activity [GO:0090681]